phosphoenolpyruvate transmembrane import into Golgi lumen [GO:1990536] (biological process) Relationships: is a type of phosphoenolpyruvate transmembrane transport [GO:0089722] References: PMID:25195688 Definition: The directed movement of phosphoenolpyruvate into the Golgi lumen across the Golgi membrane.